aldos-2-ulose dehydratase activity [GO:0033991] (molecular function) Definition: Catalysis of the reactions: 1,5-anhydro-D-fructose = 2-hydroxy-2-(hydroxymethyl)-2H-pyran-3(6H)-one + H2O; (1a) 1,5-anhydro-D-fructose = 1,5-anhydro-4-deoxy-D-glycero-hex-3-en-2-ulose + H2O and (1b) 1,5-anhydro-4-deoxy-D-glycero-hex-3-en-2-ulose = 2-hydroxy-2-(hydroxymethyl)-2H-pyran-3(6H)-one. Relationships: is a type of hydro-lyase activity [GO:0016836] Sources: EC:4.2.1.110 Also known as: 1,5-anhydro-D-fructose dehydratase (microthecin-forming) activity, 1,5-anhydro-D-fructose hydro-lyase (microthecin-forming) activity, AUDH, pyranosone dehydratase activity